{
  "gene_symbol": "TRIM40",
  "term_id": "GO:0005737",
  "gene_name": "E3 ubiquitin ligase TRIM40",
  "gene": "UniProtKB:Q6P9F5",
  "term_label": "cytoplasm"
}